{
  "gene": "UniProtKB:Q08188",
  "term_label": "Unknown cellular component",
  "gene_name": "Protein-glutamine gamma-glutamyltransferase E",
  "gene_symbol": "TGM3",
  "term_id": "UNKNOWN:0003"
}